{
  "term_label": "endocytosis",
  "gene": "UniProtKB:Q9Y6I3",
  "term_id": "GO:0006897",
  "gene_name": "Epsin-1",
  "gene_symbol": "EPN1"
}